microvillus membrane [GO:0031528] (cellular component) Subtypes: rhabdomere microvillus membrane [GO:0035997] Relationships: is a type of cell projection membrane [GO:0031253]; is part of microvillus [GO:0005902] Sources: GOC:mah Definition: The portion of the plasma membrane surrounding a microvillus.